{
  "term_label": "nucleus",
  "gene_name": "Pachytene checkpoint protein 2 homolog",
  "gene": "UniProtKB:Q15645",
  "gene_symbol": "TRIP13",
  "term_id": "GO:0005634"
}